response to pyrimidine ribonucleotide [GO:1905834] (biological process) Definition: Any process that results in a change in state or activity of a cell or an organism (in terms of movement, secretion, enzyme production, gene expression, etc.) as a result of a pyrimidine ribonucleotide stimulus. References: PMID:22065602 Sources: GOC:TermGenie, GO_REF:0000071 Subtypes: GO:1905835 Relationships: is a type of response to organophosphorus [GO:0046683]; is a type of response to nitrogen compound [GO:1901698]; is a type of GO:1901700